{
  "term_label": "DNA replication initiation",
  "gene_name": "Cell division control protein 45 homolog",
  "gene": "UniProtKB:O75419",
  "term_id": "GO:0006270",
  "gene_symbol": "CDC45"
}